{
  "gene_name": "Zinc finger protein 593",
  "gene_symbol": "ZNF593",
  "term_id": "UNKNOWN:0001",
  "gene": "UniProtKB:O00488",
  "term_label": "Unknown molecular function"
}